omega-hydroxypalmitate O-sinapoyl transferase activity [GO:0102406] (molecular function) Definition: Catalysis of the reaction: sinapoyl-CoA + 16-hydroxypalmitate = coenzyme A + 16-sinapoyloxypalmitate. Sources: EC:2.3.1.188, GOC:pz Relationships: is a type of acyltransferase activity, transferring groups other than amino-acyl groups [GO:0016747]